{
  "gene_symbol": "XPC",
  "term_label": "single-stranded DNA binding",
  "term_id": "GO:0003697",
  "gene_name": "DNA repair protein complementing XP-C cells",
  "gene": "UniProtKB:Q01831"
}